{
  "gene": "UniProtKB:P36383",
  "gene_symbol": "GJC1",
  "gene_name": "Gap junction gamma-1 protein",
  "term_label": "cell-cell signaling",
  "term_id": "GO:0007267"
}